{
  "gene_symbol": "AQP4",
  "term_label": "basolateral plasma membrane",
  "gene_name": "Aquaporin-4",
  "term_id": "GO:0016323",
  "gene": "UniProtKB:P55087"
}